K63-linked polyubiquitin modification-dependent protein binding [GO:0070530] (molecular function) References: PMID:15556404, PMID:17525341 Sources: GOC:mah Definition: Binding to a protein upon poly-ubiquitination formed by linkages between lysine residues at position 63 in the target protein. Relationships: is a type of GO:0031593